ADP deaminase activity [GO:0047629] (molecular function) Definition: Catalysis of the reaction: ADP + H2O = IDP + NH3. Sources: EC:3.5.4.7, MetaCyc:ADP-DEAMINASE-RXN Also known as: ADP aminohydrolase activity, adenosine diphosphate deaminase activity, adenosinepyrophosphate deaminase activity Relationships: is a type of adenosine-phosphate deaminase activity [GO:0047623]